{
  "gene": "UniProtKB:Q86U37",
  "gene_symbol": "LINC01551",
  "term_label": "Unknown biological process",
  "gene_name": "Uncharacterized protein encoded by LINC01551",
  "term_id": "UNKNOWN:0002"
}